{
  "term_label": "Unknown cellular component",
  "gene": "UniProtKB:Q49AS3",
  "gene_name": "Putative protein LRRC37A5P",
  "term_id": "UNKNOWN:0003",
  "gene_symbol": "LRRC37A5P"
}